{
  "gene_symbol": "ZNF766",
  "term_label": "regulation of transcription by RNA polymerase II",
  "gene_name": "Zinc finger protein 766",
  "term_id": "GO:0006357",
  "gene": "UniProtKB:Q5HY98"
}